maltose catabolic process [GO:0000025] (biological process) Sources: GOC:jl, ISBN:0198506732 Also known as: malt sugar catabolic process, malt sugar catabolism, maltose breakdown, maltose degradation, maltose hydrolysis Definition: The chemical reactions and pathways resulting in the breakdown of the disaccharide maltose (4-O-alpha-D-glucopyranosyl-D-glucopyranose). Relationships: is a type of maltose metabolic process [GO:0000023]; is a type of disaccharide catabolic process [GO:0046352]